XRCC2-RAD51D complex [GO:0033064] (cellular component) References: PMID:16093548 Sources: GOC:mah, GOC:vw Relationships: is a type of DNA recombinase mediator complex [GO:0033061]; is a type of nuclear protein-containing complex [GO:0140513] Definition: A heterodimeric DNA recombinase mediator complex that contains the Rad51 paralogs RAD51D and XRCC2, or orthologs thereof; conserved from fission yeast to human but absent from budding yeast. Also known as: DX2 complex